classical-complement-pathway C3/C5 convertase complex [GO:0005601] (cellular component) Relationships: is a type of catalytic complex [GO:1902494]; is part of extracellular space [GO:0005615] Definition: A heterodimeric protein complex that catalyzes the cleavage of complement components C3 and C5, and acts in the classical pathway of complement activation; consists of one monomer of C2a and one monomer of C4b; C2a is the catalytic subunit, but cannot catalyze cleavage alone. Sources: GOC:mah